{
  "gene_name": "PHD finger protein 10",
  "gene": "UniProtKB:Q8WUB8",
  "term_id": "GO:0004402",
  "term_label": "histone acetyltransferase activity",
  "gene_symbol": "PHF10"
}